glycerate kinase activity [GO:0008887] (molecular function) Definition: Catalysis of the reaction: D-glycerate + ATP = 3-phospho-D-glycerate + ADP + 2 H+. Also known as: ATP:(R)-glycerate 3-phosphotransferase activity, ATP:D-glycerate 2-phosphotransferase activity, D-glycerate 3-kinase activity, D-glycerate kinase activity, D-glyceric acid kinase activity, GK, glycerate kinase (phosphorylating), glycerate-3-kinase activity Sources: EC:2.7.1.31, RHEA:23516 Relationships: is a type of kinase activity [GO:0016301]; is a type of phosphotransferase activity, alcohol group as acceptor [GO:0016773]